{
  "gene_name": "Tripartite motif-containing protein 49D",
  "gene": "UniProtKB:C9J1S8",
  "gene_symbol": "TRIM49D1",
  "term_label": "ubiquitin protein ligase activity",
  "term_id": "GO:0061630"
}